{
  "term_id": "GO:0061025",
  "gene_name": "NSFL1 cofactor p47",
  "term_label": "membrane fusion",
  "gene": "UniProtKB:Q9UNZ2",
  "gene_symbol": "NSFL1C"
}